{
  "gene_symbol": "OR11H4",
  "term_id": "UNKNOWN:0003",
  "gene": "UniProtKB:Q8NGC9",
  "term_label": "Unknown cellular component",
  "gene_name": "Olfactory receptor 11H4"
}